{
  "gene": "UniProtKB:P51654",
  "term_id": "GO:0090263",
  "term_label": "positive regulation of canonical Wnt signaling pathway",
  "gene_name": "Glypican-3",
  "gene_symbol": "GPC3"
}